limit dextrinase activity [GO:0010303] (molecular function) Relationships: is a type of hydrolase activity, hydrolyzing O-glycosyl compounds [GO:0004553] Definition: Catalysis of the hydrolysis of (1,6)-alpha-D-glucosidic linkages in alpha- and beta-limit dextrins of amylopectin and glycogen, and in amylopectin and pullulan. Sources: EC:3.2.1.142 Also known as: R-enzyme, amylopectin-1,6-glucosidase activity, dextrin alpha-1,6-glucanohydrolase activity